{
  "term_label": "Unknown biological process",
  "gene_name": "Basic salivary proline-rich protein 4",
  "gene": "UniProtKB:P10163",
  "term_id": "UNKNOWN:0002",
  "gene_symbol": "PRB4"
}